{
  "gene_symbol": "CTAGE15",
  "gene_name": "cTAGE family member 15",
  "term_id": "UNKNOWN:0001",
  "term_label": "Unknown molecular function",
  "gene": "UniProtKB:A4D2H0"
}